{
  "term_id": "GO:0006307",
  "gene_name": "Alpha-ketoglutarate-dependent dioxygenase FTO",
  "term_label": "DNA alkylation repair",
  "gene_symbol": "FTO",
  "gene": "UniProtKB:Q9C0B1"
}